{
  "term_id": "UNKNOWN:0001",
  "gene": "UniProtKB:Q6UW68",
  "term_label": "Unknown molecular function",
  "gene_symbol": "TMEM205",
  "gene_name": "Transmembrane protein 205"
}